regulation of heterotypic cell-cell adhesion [GO:0034114] (biological process) Subtypes: GO:0034115, positive regulation of heterotypic cell-cell adhesion [GO:0034116], regulation of platelet rolling [GO:0160017] Sources: GOC:add Relationships: is a type of regulation of cell-cell adhesion [GO:0022407]; regulates heterotypic cell-cell adhesion [GO:0034113] Definition: Any process that modulates the frequency, rate, or extent of heterotypic cell-cell adhesion.